{
  "gene_symbol": "CBLN3",
  "gene_name": "Cerebellin-3",
  "term_id": "GO:0099558",
  "gene": "UniProtKB:Q6UW01",
  "term_label": "maintenance of synapse structure"
}